{
  "gene": "UniProtKB:Q01105",
  "gene_name": "Protein SET",
  "term_label": "Unknown biological process",
  "term_id": "UNKNOWN:0002",
  "gene_symbol": "SET"
}